{
  "term_label": "mitochondrial tryptophanyl-tRNA aminoacylation",
  "gene": "UniProtKB:Q9UGM6",
  "gene_symbol": "WARS2",
  "gene_name": "Tryptophan--tRNA ligase, mitochondrial",
  "term_id": "GO:0070183"
}